{
  "term_id": "GO:0016020",
  "gene_symbol": "ARL6IP1",
  "gene_name": "ADP-ribosylation factor-like protein 6-interacting protein 1",
  "gene": "UniProtKB:Q15041",
  "term_label": "membrane"
}